{
  "term_id": "GO:0043005",
  "term_label": "neuron projection",
  "gene_symbol": "HTR3A",
  "gene": "UniProtKB:P46098",
  "gene_name": "5-hydroxytryptamine receptor 3A"
}